{
  "term_id": "GO:0002767",
  "gene_symbol": "LAIR2",
  "gene": "UniProtKB:Q6ISS4",
  "gene_name": "Leukocyte-associated immunoglobulin-like receptor 2",
  "term_label": "immune response-inhibiting cell surface receptor signaling pathway"
}